low-density lipoprotein particle mediated signaling [GO:0055096] (biological process) Definition: The series of molecular signals mediated by the detection of low-density lipoprotein particle. Relationships: is a type of lipoprotein particle mediated signaling [GO:0055095]; is part of cellular response to low-density lipoprotein particle stimulus [GO:0071404] Also known as: low-density lipoprotein mediated signalling, low-density lipoprotein particle mediated signal transduction, low-density lipoprotein particle-mediated signaling References: PMID:16013438 Sources: GOC:BHF, GOC:rl